{
  "gene": "UniProtKB:Q00975",
  "term_label": "voltage-gated calcium channel complex",
  "gene_symbol": "CACNA1B",
  "gene_name": "Voltage-dependent N-type calcium channel subunit alpha-1B",
  "term_id": "GO:0005891"
}